red chlorophyll catabolite reductase activity [GO:0051743] (molecular function) References: PMID:10743659 Relationships: is a type of oxidoreductase activity, acting on the CH-CH group of donors, iron-sulfur protein as acceptor [GO:0016636] Also known as: RCC reductase activity Definition: Catalysis of the reaction: red chlorophyll catabolite + reduced ferredoxin + 2 H+ = primary fluorescent catabolite + oxidized ferredoxin. This reaction is the reduction of the C20/C1 double bond in the pyrrole system of red chlorophyll catabolite (RCC) to a colorless tetrapyrrole (pFCC) with a strong blue fluorescence.